{
  "gene": "UniProtKB:P22680",
  "term_id": "UNKNOWN:0003",
  "gene_symbol": "CYP7A1",
  "gene_name": "Cytochrome P450 7A1",
  "term_label": "Unknown cellular component"
}